{
  "gene_symbol": "MTREX",
  "gene": "UniProtKB:P42285",
  "gene_name": "Exosome RNA helicase MTR4",
  "term_id": "GO:0006401",
  "term_label": "RNA catabolic process"
}